{
  "term_label": "gluconeogenesis",
  "gene_name": "Triosephosphate isomerase",
  "gene": "UniProtKB:P60174",
  "gene_symbol": "TPI1",
  "term_id": "GO:0006094"
}